{
  "term_label": "olfactory receptor activity",
  "gene_symbol": "OR6C4",
  "gene": "UniProtKB:Q8NGE1",
  "gene_name": "Olfactory receptor 6C4",
  "term_id": "GO:0004984"
}